{
  "gene": "UniProtKB:Q9H4L7",
  "term_label": "DNA binding",
  "gene_symbol": "SMARCAD1",
  "term_id": "GO:0003677",
  "gene_name": "SWI_SNF-related matrix-associated actin-dependent regulator of chromatin subfamily A containing DEAD_H box 1"
}